{
  "gene_name": "Protein SET",
  "term_label": "histone binding",
  "term_id": "GO:0042393",
  "gene_symbol": "SET",
  "gene": "UniProtKB:Q01105"
}